{
  "term_label": "troponin I binding",
  "gene": "UniProtKB:P45378",
  "term_id": "GO:0031013",
  "gene_name": "Troponin T, fast skeletal muscle",
  "gene_symbol": "TNNT3"
}